{
  "term_label": "Unknown biological process",
  "gene": "UniProtKB:Q86T29",
  "gene_symbol": "ZNF605",
  "term_id": "UNKNOWN:0002",
  "gene_name": "Zinc finger protein 605"
}